regulation of protein oligomerization [GO:0032459] (biological process) Sources: GOC:mah Definition: Any process that modulates the frequency, rate or extent of protein oligomerization. Subtypes: GO:0032460, positive regulation of protein oligomerization [GO:0032461], regulation of protein homooligomerization [GO:0032462], regulation of protein tetramerization [GO:1901090] Relationships: is a type of regulation of protein-containing complex assembly [GO:0043254]; regulates GO:0051259